{
  "term_id": "GO:0003682",
  "gene_name": "Bromodomain-containing protein 2",
  "term_label": "chromatin binding",
  "gene_symbol": "BRD2",
  "gene": "UniProtKB:P25440"
}